{
  "gene_name": "Small nuclear protein PRAC1",
  "gene_symbol": "PRAC1",
  "gene": "UniProtKB:Q96KF2",
  "term_label": "nucleoplasm",
  "term_id": "GO:0005654"
}